L-dopa biosynthetic process [GO:1903185] (biological process) Definition: The chemical reactions and pathways resulting in the formation of L-dopa. Also known as: L-dopa anabolism, L-dopa biosynthesis, L-dopa formation, L-dopa synthesis Regulation: regulated by regulation of L-dopa biosynthetic process [GO:1903195]; negatively regulated by negative regulation of L-dopa biosynthetic process [GO:1903196]; positively regulated by positive regulation of L-dopa biosynthetic process [GO:1903197] Relationships: is_a GO:0009073; is a type of modified amino acid biosynthetic process [GO:0042398]; is a type of L-amino acid biosynthetic process [GO:0170034]; is a type of non-proteinogenic amino acid biosynthetic process [GO:0170043]; is a type of L-dopa metabolic process [GO:1903184] References: PMID:8822146 Sources: GOC:PARL, GOC:TermGenie, GOC:bf, GO_REF:0000068